{
  "term_label": "calcium-dependent phospholipid binding",
  "gene_symbol": "SYT15B",
  "gene_name": "Synaptotagmin-15B",
  "term_id": "GO:0005544",
  "gene": "UniProtKB:X6R8R1"
}